positive regulation of mRNA 3'-end processing [GO:0031442] (biological process) Subtypes: positive regulation of mRNA alternative polyadenylation [GO:0140409] Also known as: up regulation of mRNA 3'-end processing, up-regulation of mRNA 3'-end processing, upregulation of mRNA 3'-end processing, activation of mRNA 3'-end processing, stimulation of mRNA 3'-end processing Relationships: is a type of regulation of mRNA 3'-end processing [GO:0031440]; is a type of GO:0050685; positively regulates GO:0031124 Sources: GOC:mah Definition: Any process that activates or increases the frequency, rate or extent of mRNA 3'-end processing.